regulation of 17-methylnonadec-1-ene biosynthetic process [GO:1900956] (biological process) Definition: Any process that modulates the frequency, rate or extent of 17-methylnonadec-1-ene biosynthetic process. Sources: GOC:TermGenie, GOC:mengo_curators Also known as: regulation of 17-methylnonadec-1-ene anabolism, regulation of 17-methylnonadec-1-ene biosynthesis, regulation of 17-methylnonadec-1-ene formation, regulation of 17-methylnonadec-1-ene synthesis Relationships: is a type of regulation of olefin biosynthetic process [GO:1900911]; regulates 17-methylnonadec-1-ene biosynthetic process [GO:1900883] Subtypes: negative regulation of 17-methylnonadec-1-ene biosynthetic process [GO:1900957], positive regulation of 17-methylnonadec-1-ene biosynthetic process [GO:1900958]